cellulose synthase activity [GO:0016759] (MF) Also known as: cellulose synthetase activity Definition: Catalysis of the reaction: nucleoside-disphosphate-glucose + ((1,4)-beta-D-glucosyl)(n) = nucleoside-disphosphate + ((1,4)-beta-D-glucosyl)(n+1). Relationships: is a type of GO:0046527 Subtypes: cellulose synthase (UDP-forming) activity [GO:0016760], cellulose synthase (GDP-forming) activity [GO:0016761] Sources: GOC:curators